response to clopidogrel [GO:1903493] (biological process) Relationships: is a type of response to nitrogen compound [GO:1901698]; is a type of response to oxygen-containing compound [GO:1901700] References: PMID:23392654 Sources: GOC:TermGenie, GO_REF:0000071 Definition: Any process that results in a change in state or activity of a cell or an organism (in terms of movement, secretion, enzyme production, gene expression, etc.) as a result of a clopidogrel stimulus. Clopidogrel is a is an oral, thienopyridine-class antiplatelet agent used to inhibit blood clots in coronary artery disease, peripheral vascular disease, and cerebrovascular disease.